positive regulation of mesonephric glomerular mesangial cell proliferation [GO:2000092] (biological process) Definition: Any process that activates or increases the frequency, rate or extent of mesonephric glomerular mesangial cell proliferation. Relationships: is a type of positive regulation of glomerular mesangial cell proliferation [GO:0072126]; is a type of regulation of mesonephric glomerular mesangial cell proliferation [GO:2000090]; is a type of positive regulation of cell proliferation involved in mesonephros development [GO:2000608]; positively regulates GO:0061269 Sources: GOC:mtg_kidney_jan10